homogentisate 1,2-dioxygenase activity [GO:0004411] (molecular function) Also known as: homogentisate dioxygenase activity, homogentisate oxidase activity, homogentisate oxygenase activity, homogentisate:oxygen 1,2-oxidoreductase (decyclizing), homogentisic acid oxidase activity, homogentisic acid oxygenase activity, homogentisic oxygenase activity, homogentisicase activity Relationships: is a type of oxidoreductase activity, acting on single donors with incorporation of molecular oxygen, incorporation of two atoms of oxygen [GO:0016702] Sources: EC:1.13.11.5, RHEA:15449 Definition: Catalysis of the reaction: homogentisate + O2 = 4-maleylacetoacetate + H+.